{
  "term_id": "UNKNOWN:0003",
  "gene_name": "Keratin-associated protein 19-7",
  "gene_symbol": "KRTAP19-7",
  "gene": "UniProtKB:Q3SYF9",
  "term_label": "Unknown cellular component"
}